{
  "gene_name": "Mucin-3A",
  "gene_symbol": "MUC3A",
  "term_id": "UNKNOWN:0001",
  "term_label": "Unknown molecular function",
  "gene": "UniProtKB:Q02505"
}